leukotriene C4 gamma-glutamyl transferase activity [GO:0103068] (molecular function) Relationships: is a type of GO:0016755 Definition: Catalysis of the reaction: leukotriene C4 + a standard alpha amino acid = leukotriene D4 + an (gamma-L-glutamyl)-L-amino acid. References: PMID:1676842, PMID:9139674 Sources: GOC:pz